{
  "gene_name": "Transmembrane channel-like protein 7",
  "term_label": "Unknown cellular component",
  "gene": "UniProtKB:Q7Z402",
  "term_id": "UNKNOWN:0003",
  "gene_symbol": "TMC7"
}